{
  "gene_symbol": "SLC22A3",
  "gene": "UniProtKB:O75751",
  "gene_name": "Solute carrier family 22 member 3",
  "term_id": "GO:0015695",
  "term_label": "organic cation transport"
}